{
  "term_id": "GO:0010314",
  "gene_name": "Ventricular zone-expressed PH domain-containing protein homolog 1",
  "gene": "UniProtKB:Q14D04",
  "gene_symbol": "VEPH1",
  "term_label": "phosphatidylinositol-5-phosphate binding"
}